histone benzoyllysine debenzoylase activity [GO:0140228] (molecular function) Relationships: is a type of histone modifying activity [GO:0140993] Definition: Catalysis of the reaction: N(6)-benzoyl-L-lysyl-[protein] + NAD+ + H2O = 2''-O-benzoyl-ADP-D-ribose + nicotinamide + L-lysyl-[protein]. References: PMID:34961760